rod spherule [GO:0044317] (cellular component) References: PMID:26930660 Definition: A specialized neuron projection which is the site of synaptic transmission produced by retinal rod cells. Rod spherules are small round enlargements of the axon (3-5 micrometers diameter) or even extensions of the cell body. Also known as: rod cell spherule, rod photoreceptor spherule Relationships: is a type of neuron projection [GO:0043005]